{
  "gene_name": "TBC1 domain family member 5",
  "gene": "UniProtKB:Q92609",
  "term_label": "endosome membrane",
  "gene_symbol": "TBC1D5",
  "term_id": "GO:0010008"
}